{
  "gene": "UniProtKB:P17026",
  "term_id": "GO:0005634",
  "gene_symbol": "ZNF22",
  "gene_name": "Zinc finger protein 22",
  "term_label": "nucleus"
}